intranuclear rod [GO:0061836] (cellular component) Also known as: intranuclear actin rod Relationships: is a type of supramolecular fiber [GO:0099512] Definition: A macromolecular fiber consisting of actin and cofilin that is formed in the nucleus as a consequence of chemical or mechanical stress conditions. References: PMID:28074884